{
  "gene_symbol": "RUNDC3A",
  "gene": "UniProtKB:Q59EK9",
  "term_label": "Unknown biological process",
  "gene_name": "RUN domain-containing protein 3A",
  "term_id": "UNKNOWN:0002"
}